{
  "gene": "UniProtKB:Q86VW0",
  "term_label": "Unknown biological process",
  "gene_symbol": "SESTD1",
  "term_id": "UNKNOWN:0002",
  "gene_name": "SEC14 domain and spectrin repeat-containing protein 1"
}